{
  "gene": "UniProtKB:P0CG38",
  "gene_name": "POTE ankyrin domain family member I",
  "gene_symbol": "POTEI",
  "term_label": "protein kinase binding",
  "term_id": "GO:0019901"
}